sugar-terminal-phosphatase activity [GO:0050309] (molecular function) Subtypes: glucose-6-phosphatase activity [GO:0004346] Sources: EC:3.1.3.58 Also known as: sugar-omega-phosphate phosphohydrolase activity, xylitol-5-phosphatase activity Relationships: is a type of sugar-phosphatase activity [GO:0050308] Definition: Catalysis of the reaction: H2O + sugar phosphorylated on the terminal carbon = a sugar + phosphate.